{
  "gene_symbol": "KHSRP",
  "gene_name": "Far upstream element-binding protein 2",
  "term_label": "nucleus",
  "gene": "UniProtKB:Q92945",
  "term_id": "GO:0005634"
}